{
  "gene_name": "Chloride intracellular channel protein 2",
  "gene": "UniProtKB:O15247",
  "term_label": "chloride channel activity",
  "term_id": "GO:0005254",
  "gene_symbol": "CLIC2"
}